{
  "gene_name": "Homeobox protein DLX-4",
  "term_label": "cell differentiation",
  "gene_symbol": "DLX4",
  "gene": "UniProtKB:Q92988",
  "term_id": "GO:0030154"
}